prenyl-FMNH2 biosynthetic process [GO:0120232] (biological process) Definition: The chemical reactions and pathways resulting in prenyl-FMNH2, an essential cofactor for the decarboxylase enzymes UbiD and Fdc1. References: PMID:25647642, PMID:26083743, PMID:26083754 Sources: GOC:krc Relationships: is a type of ribonucleoside monophosphate biosynthetic process [GO:0009156]; is_a ribonucleotide biosynthetic process [GO:0009260]; is a type of GO:0042727 Also known as: prenyl-FMNH2 anabolism, prenyl-FMNH2 biosynthesis, prenyl-FMNH2 formation, prenyl-FMNH2 synthesis, prenylated FMNH2 anabolism, prenylated FMNH2 biosynthesis, prenylated FMNH2 biosynthetic process, prenylated FMNH2 formation, prenylated FMNH2 synthesis